T cell extravasation [GO:0072683] (biological process) Regulation: regulated by regulation of T cell extravasation [GO:2000407]; negatively regulated by GO:2000408; positively regulated by positive regulation of T cell extravasation [GO:2000409] Subtypes: memory T cell extravasation [GO:0035683], helper T cell extravasation [GO:0035684], CD8-positive, alpha-beta T cell extravasation [GO:0035697] Relationships: is a type of cellular extravasation [GO:0045123]; is a type of T cell migration [GO:0072678] Definition: The migration of a T cell from the blood vessels into the surrounding tissue. Sources: CL:0000084, GOC:BHF, GOC:mah Also known as: T lymphocyte extravasation, T-cell extravasation, T-lymphocyte extravasation